{
  "term_id": "GO:0005737",
  "gene": "UniProtKB:Q9Y5K6",
  "gene_symbol": "CD2AP",
  "gene_name": "CD2-associated protein",
  "term_label": "cytoplasm"
}